neuron cell-cell adhesion [GO:0007158] (biological process) Relationships: is a type of cell-cell adhesion [GO:0098609] Also known as: neuron adhesion, neuronal cell adhesion Definition: The attachment of a neuron to another cell via adhesion molecules. Sources: GOC:go_curators